{
  "term_id": "GO:0000922",
  "term_label": "spindle pole",
  "gene_name": "Centrosomal protein of 19 kDa",
  "gene_symbol": "CEP19",
  "gene": "UniProtKB:Q96LK0"
}